{
  "gene": "UniProtKB:P05023",
  "term_id": "GO:0042383",
  "gene_name": "Sodium_potassium-transporting ATPase subunit alpha-1",
  "gene_symbol": "ATP1A1",
  "term_label": "sarcolemma"
}